malonic acid import across plasma membrane [GO:0098715] (biological process) Relationships: is a type of import across plasma membrane [GO:0098739]; is a type of malonic acid transmembrane transport [GO:1901553] Sources: GOC:dos Also known as: malonate import into cell, malonic acid import into cell Definition: The directed movement of malonic acid from outside of a cell, across the plasma membrane and into the cytosol.